{
  "gene": "UniProtKB:Q9Y3Z3",
  "gene_name": "Deoxynucleoside triphosphate triphosphohydrolase SAMHD1",
  "gene_symbol": "SAMHD1",
  "term_id": "GO:0051607",
  "term_label": "defense response to virus"
}